adenosine-tetraphosphatase activity [GO:0047624] (molecular function) Also known as: adenosine-tetraphosphate phosphohydrolase activity Relationships: is a type of pyrophosphatase activity [GO:0016462] Sources: EC:3.6.1.14, MetaCyc:ADENOSINE-TETRAPHOSPHATASE-RXN Definition: Catalysis of the reaction: adenosine 5'-tetraphosphate + H2O = ATP + phosphate.